{
  "gene_name": "Ligand-dependent nuclear receptor-interacting factor 1",
  "gene": "UniProtKB:Q5T3J3",
  "gene_symbol": "LRIF1",
  "term_label": "Unknown molecular function",
  "term_id": "UNKNOWN:0001"
}